{
  "term_id": "GO:0055064",
  "term_label": "chloride ion homeostasis",
  "gene_symbol": "SLC12A9",
  "gene": "UniProtKB:Q9BXP2",
  "gene_name": "Solute carrier family 12 member 9"
}